D3 dopamine receptor binding [GO:0031750] (molecular function) Also known as: D3 dopamine receptor ligand Relationships: is a type of dopamine receptor binding [GO:0050780] Sources: GOC:mah, GOC:nln Definition: Binding to a D3 dopamine receptor.